RNA capping [GO:0036260] (biological process) Definition: The sequence of enzymatic reactions by which a cap structure is added to the 5' end of nascent RNA polymerase transcripts. Examples of RNA capping include 7-methyl-G caps found on all RNA polymerase II transcripts and nucleotide-containing cofactor caps, such as NAD(H) or FAD, found on bacterial trancripts. References: PMID:18775984, PMID:27383794, PMID:29681497, PMID:30353673 Sources: GOC:bf, GOC:krc, GOC:mah Relationships: is a type of RNA 5'-end processing [GO:0000966] Subtypes: 7-methylguanosine RNA capping [GO:0009452], 7-methylguanosine cap hypermethylation [GO:0036261], GO:0180031, snRNA 2,2,7-trimethylguanosine (TMG) capping [GO:1990273]